S-acyltransferase activity [GO:0016417] (molecular function) Definition: Catalysis of the transfer of an acyl group to a sulfur atom on the acceptor molecule. Subtypes: S-acetyltransferase activity [GO:0016418], GO:0016419, S-succinyltransferase activity [GO:0016751], protein-cysteine S-acyltransferase activity [GO:0019707] Sources: GOC:ai Relationships: is a type of acyltransferase activity, transferring groups other than amino-acyl groups [GO:0016747]